{
  "term_id": "GO:0051260",
  "gene_name": "Atlastin-3",
  "gene_symbol": "ATL3",
  "gene": "UniProtKB:Q6DD88",
  "term_label": "protein homooligomerization"
}